{
  "gene_name": "Aromatic-L-amino-acid decarboxylase",
  "term_label": "catecholamine metabolic process",
  "gene_symbol": "DDC",
  "gene": "UniProtKB:P20711",
  "term_id": "GO:0006584"
}